acetylcholine receptor signaling pathway [GO:0095500] (biological process) Subtypes: GO:0007213 Definition: The series of molecular signals generated as a consequence of an acetylcholine receptor binding to one of its physiological ligands. Sources: GOC:mah Relationships: is a type of postsynaptic signal transduction [GO:0098926]; is part of cellular response to acetylcholine [GO:1905145]; has part acetylcholine receptor activity [GO:0015464] Also known as: acetylcholine receptor signalling pathway